dorsal aorta morphogenesis [GO:0035912] (biological process) Relationships: is a type of aorta morphogenesis [GO:0035909]; BFO_0000050 dorsal aorta development [GO:0035907] Sources: GOC:bf, GOC:dgh, UBERON:0005805, Wikipedia:Aorta, ZFA:0000014 Definition: The process in which the anatomical structures of the dorsal aorta are generated and organized. The dorsal aorta is a blood vessel in a single-pass circulatory system that carries oxygenated blood from the gills to the rest of the body. In a single-pass circulatory system blood passes once through the heart to supply the body once.